{
  "gene": "UniProtKB:Q10570",
  "gene_name": "Cleavage and polyadenylation specificity factor subunit 1",
  "term_label": "Unknown molecular function",
  "gene_symbol": "CPSF1",
  "term_id": "UNKNOWN:0001"
}